trypanothione metabolic process [GO:0046206] (BP) Also known as: trypanothione metabolism Definition: The chemical reactions and pathways involving trypanothione (N1,N6,-bis(glutathionyl)spermidine), an essential redox intermediate in intracellular thiol redox regulation which also plays a role in protecting against oxidative stress. Sources: GOC:ai Subtypes: GO:0019342, trypanothione catabolic process [GO:0046207] Relationships: is a type of GO:0006790